{
  "term_id": "GO:0035196",
  "gene_symbol": "SNIP1",
  "gene": "UniProtKB:Q8TAD8",
  "term_label": "miRNA processing",
  "gene_name": "Smad nuclear-interacting protein 1"
}